{
  "gene": "UniProtKB:Q5JTD7",
  "gene_symbol": "LRRC73",
  "term_label": "Unknown biological process",
  "gene_name": "Leucine-rich repeat-containing protein 73",
  "term_id": "UNKNOWN:0002"
}